{
  "gene": "UniProtKB:P43119",
  "term_id": "GO:0005886",
  "term_label": "plasma membrane",
  "gene_symbol": "PTGIR",
  "gene_name": "Prostacyclin receptor"
}